{
  "term_id": "GO:0042393",
  "gene_symbol": "HJURP",
  "term_label": "histone binding",
  "gene_name": "Holliday junction recognition protein",
  "gene": "UniProtKB:Q8NCD3"
}